{
  "term_id": "UNKNOWN:0003",
  "gene_symbol": "TMEM62",
  "gene_name": "Transmembrane protein 62",
  "gene": "UniProtKB:Q0P6H9",
  "term_label": "Unknown cellular component"
}